{
  "gene_name": "Cancer_testis antigen 1",
  "gene_symbol": "CTAG1A",
  "gene": "UniProtKB:P78358",
  "term_label": "tRNA threonylcarbamoyladenosine metabolic process",
  "term_id": "GO:0070525"
}